{
  "gene_name": "Phosphatidylinositol 4,5-bisphosphate 5-phosphatase A",
  "term_id": "GO:0043005",
  "gene": "UniProtKB:Q15735",
  "gene_symbol": "INPP5J",
  "term_label": "neuron projection"
}